rDNA chromatin condensation [GO:0070550] (biological process) Definition: The process in which the chromatin structure of the rDNA repeats is compacted. In S. cerevisiae, condensation and resolution of the rDNA occurs during anaphase. References: PMID:10811823, PMID:15137940 Sources: GOC:dgf Also known as: rDNA condensation, rDNA packaging Relationships: is a type of chromosome condensation [GO:0030261]; BFO_0000050 GO:1990700